{
  "term_label": "phosphate ion transmembrane transport",
  "gene_name": "Sodium-dependent phosphate transporter 1",
  "term_id": "GO:0035435",
  "gene": "UniProtKB:Q8WUM9",
  "gene_symbol": "SLC20A1"
}